{
  "term_id": "GO:0005740",
  "term_label": "mitochondrial envelope",
  "gene": "UniProtKB:O43772",
  "gene_name": "Mitochondrial carnitine_acylcarnitine carrier protein",
  "gene_symbol": "SLC25A20"
}